{
  "term_id": "GO:0005615",
  "gene_name": "Kallikrein-5",
  "gene": "UniProtKB:Q9Y337",
  "gene_symbol": "KLK5",
  "term_label": "extracellular space"
}